angiotensin receptor binding [GO:0031701] (molecular function) Relationships: is_a G protein-coupled receptor binding [GO:0001664] Definition: Binding to an angiotensin receptor. Also known as: angiotensin receptor ligand Sources: GOC:mah, GOC:nln Subtypes: GO:0031702, type 2 angiotensin receptor binding [GO:0031703]